{
  "term_id": "GO:0000981",
  "gene_name": "Cyclic AMP-responsive element-binding protein 5",
  "gene": "UniProtKB:Q02930",
  "gene_symbol": "CREB5",
  "term_label": "DNA-binding transcription factor activity, RNA polymerase II-specific"
}